{
  "term_id": "UNKNOWN:0003",
  "term_label": "Unknown cellular component",
  "gene": "UniProtKB:P05813",
  "gene_symbol": "CRYBA1",
  "gene_name": "Beta-crystallin A3"
}